{
  "term_id": "UNKNOWN:0001",
  "term_label": "Unknown molecular function",
  "gene": "UniProtKB:Q6NSI8",
  "gene_symbol": "SANBR",
  "gene_name": "SANT and BTB domain regulator of class switch recombination"
}